{
  "gene": "UniProtKB:Q9BTX1",
  "term_label": "nuclear pore organization",
  "gene_name": "Nucleoporin NDC1",
  "term_id": "GO:0006999",
  "gene_symbol": "NDC1"
}